{
  "term_id": "GO:0008330",
  "gene": "UniProtKB:Q99956",
  "term_label": "protein tyrosine/threonine phosphatase activity",
  "gene_name": "Dual specificity protein phosphatase 9",
  "gene_symbol": "DUSP9"
}